anterior neural tube closure [GO:0061713] (biological process) Relationships: is a type of tube closure [GO:0060606]; is part of neural tube closure [GO:0001843] References: PMID:17286298 Sources: GOC:BHF, GOC:dph, GOC:hal Definition: The step in the formation of the neural tube, where the paired anterior neural folds are brought together and fuse at the dorsal midline.